{
  "term_label": "Unknown cellular component",
  "term_id": "UNKNOWN:0003",
  "gene_symbol": "ANKRD36B",
  "gene_name": "Ankyrin repeat domain-containing protein 36B",
  "gene": "UniProtKB:Q8N2N9"
}